low-affinity D-glucose:proton symporter activity [GO:0005359] (molecular function) Definition: Enables the transfer of a solute or solutes from one side of a membrane to the other according to the reaction: glucose(out) + H(out)+ = glucose(in) + H(in)+. In low-affinity transport the transporter is able to bind the solute only if it is present at very high concentrations. Symporter activity enables the active transport of a solute across a membrane by a mechanism whereby two or more species are transported together in the same direction in a tightly coupled process not directly linked to a form of energy other than chemiosmotic energy. Relationships: is a type of GO:0005356 Sources: GOC:mtg_transport Also known as: low-affinity hydrogen/glucose transporter activity, low-affinity hydrogen:glucose transporter activity, low-affinity glucose:proton symporter activity, low-affinity hydrogen:glucose symporter activity